{
  "term_label": "semaphorin-plexin signaling pathway",
  "gene": "UniProtKB:Q9Y4D7",
  "term_id": "GO:0071526",
  "gene_name": "Plexin-D1",
  "gene_symbol": "PLXND1"
}